methenyltetrahydromethanopterin cyclohydrolase activity [GO:0018759] (molecular function) Sources: EC:3.5.4.27, RHEA:19053 Relationships: is a type of cyclohydrolase activity [GO:0019238] Also known as: 5,10-methenyltetrahydromethanopterin 10-hydrolase (decyclizing), 5,10-methenyltetrahydromethanopterin cyclohydrolase activity, N5,N10-methenyltetrahydromethanopterin cyclohydrolase activity, methenyl-H(4)MPT cyclohydrolase activity, methenyl-H4MPT cyclohydrolase activity Definition: Catalysis of the reaction: 5,10-methenyl-5,6,7,8-tetrahydromethanopterin + H2O = N(5)-formyl-5,6,7,8-tetrahydromethanopterin + H+.